internal genitalia morphogenesis [GO:0035260] (biological process) References: PMID:24793987, PMID:25247640 Relationships: is_a GO:0035112 Definition: The process in which the anatomical structures of the internal genitalia are generated and organized. The internal genitalia are the internal sex organs such as the uterine tube, the uterus and the vagina in female mammals, and the testis, seminal vesicle, ejaculatory duct and prostate in male mammals.